thiamine diphosphate metabolic process [GO:0042357] (biological process) Relationships: is a type of phosphate-containing compound metabolic process [GO:0006796]; is a type of organophosphate metabolic process [GO:0019637]; is a type of thiamine-containing compound metabolic process [GO:0042723] Definition: The chemical reactions and pathways involving thiamine diphosphate, a derivative of thiamine (vitamin B1) which acts as a coenzyme in a range of processes including the Krebs cycle. Also known as: TPP metabolic process, TPP metabolism, thiamin diphosphate metabolic process, thiamin diphosphate metabolism, thiamin pyrophosphate metabolic process, thiamin pyrophosphate metabolism, thiamine diphosphate metabolism, thiamine pyrophosphate metabolic process, thiamine pyrophosphate metabolism Sources: GOC:jl, ISBN:0198506732 Subtypes: thiamine diphosphate biosynthetic process [GO:0009229], thiamine diphosphate catabolic process [GO:0042358], GO:0042370